{
  "gene": "UniProtKB:P0C7W9",
  "gene_name": "Putative protein FAM90A14",
  "term_id": "UNKNOWN:0002",
  "gene_symbol": "FAM90A14",
  "term_label": "Unknown biological process"
}